{
  "term_label": "regulation of transcription by RNA polymerase II",
  "gene_name": "HMG box-containing protein 1",
  "term_id": "GO:0006357",
  "gene": "UniProtKB:O60381",
  "gene_symbol": "HBP1"
}